sulfurated eukaryotic molybdenum cofactor(2-) biosynthetic process [GO:1902756] (BP) References: PMID:18258600 Sources: GOC:TermGenie, GOC:dph, GO_REF:0000068 Relationships: is_a phosphorus metabolic process [GO:0006793]; is a type of biosynthetic process [GO:0009058]; has part GO:0008265 Also known as: sulfurated eukaryotic molybdenum cofactor(2-) anabolism, sulfurated eukaryotic molybdenum cofactor(2-) biosynthesis, sulfurated eukaryotic molybdenum cofactor(2-) formation, sulfurated eukaryotic molybdenum cofactor(2-) synthesis Definition: The chemical reactions and pathways resulting in the formation of sulfurated eukaryotic molybdenum cofactor(2-).